{
  "term_id": "GO:0070840",
  "term_label": "dynein complex binding",
  "gene": "UniProtKB:Q9UKB1",
  "gene_name": "F-box_WD repeat-containing protein 11",
  "gene_symbol": "FBXW11"
}